{
  "gene_symbol": "C21orf140",
  "term_id": "UNKNOWN:0001",
  "term_label": "Unknown molecular function",
  "gene_name": "Uncharacterized protein C21orf140",
  "gene": "UniProtKB:B9A014"
}